tetrahydrodipicolinate N-acetyltransferase activity [GO:0047200] (molecular function) Also known as: acetyl-CoA:(S)-2,3,4,5-tetrahydrodipicolinate-2,6-dicarboxylate N2-acetyltransferase activity, acetyl-CoA:(S)-2,3,4,5-tetrahydropyridine-2,6-dicarboxylate 2-N-acetyltransferase activity, acetyl-CoA:L-2,3,4,5-tetrahydrodipicolinate N2-acetyltransferase activity, tetrahydrodipicolinate acetylase activity, tetrahydrodipicolinate:acetyl-CoA acetyltransferase activity Relationships: is a type of GO:0008080 Sources: EC:2.3.1.89, RHEA:13085 Definition: Catalysis of the reaction: (S)-2,3,4,5-tetrahydrodipicolinate + acetyl-CoA + H2O = L-2-acetamido-6-oxopimelate + CoA.